{
  "gene_name": "Transmembrane and coiled-coil domains protein 1",
  "term_id": "GO:0097750",
  "gene": "UniProtKB:O94876",
  "term_label": "endosome membrane tubulation",
  "gene_symbol": "TMCC1"
}